{
  "term_label": "Unknown biological process",
  "gene_name": "Glycine N-acyltransferase-like protein 2",
  "gene": "UniProtKB:Q8WU03",
  "term_id": "UNKNOWN:0002",
  "gene_symbol": "GLYATL2"
}